{
  "term_label": "cytokine activity",
  "term_id": "GO:0005125",
  "gene_symbol": "IL20",
  "gene_name": "Interleukin-20",
  "gene": "UniProtKB:Q9NYY1"
}